{
  "term_id": "UNKNOWN:0002",
  "gene": "UniProtKB:P26436",
  "term_label": "Unknown biological process",
  "gene_symbol": "ACRV1",
  "gene_name": "Acrosomal protein SP-10"
}